{
  "gene_name": "Protein BANP",
  "gene": "UniProtKB:Q8N9N5",
  "term_id": "UNKNOWN:0002",
  "term_label": "Unknown biological process",
  "gene_symbol": "BANP"
}